{
  "term_id": "GO:0005694",
  "gene": "UniProtKB:P54132",
  "gene_symbol": "BLM",
  "term_label": "chromosome",
  "gene_name": "RecQ-like DNA helicase BLM"
}